{
  "gene": "UniProtKB:O95989",
  "term_id": "GO:0008486",
  "gene_name": "Diphosphoinositol polyphosphate phosphohydrolase 1",
  "term_label": "diphosphoinositol-polyphosphate diphosphatase activity",
  "gene_symbol": "NUDT3"
}